{
  "term_label": "tube formation",
  "gene_symbol": "SDCCAG8",
  "gene": "UniProtKB:Q86SQ7",
  "term_id": "GO:0035148",
  "gene_name": "Serologically defined colon cancer antigen 8"
}